detoxification of mercury ion [GO:0050787] (biological process) References: PMID:10774920 Definition: Any process that reduce or remove the toxicity of mercuric ion. These include transport of mercury away from sensitive areas and to compartments or complexes whose purpose is sequestration of mercury ion and/or reduction of mercury ion (Hg[II]) to metallic mercury (Hg[0]). Relationships: is a type of detoxification of inorganic compound [GO:0061687]; is part of response to mercury ion [GO:0046689]